{
  "gene_name": "Putative uncharacterized protein ASB16-AS1",
  "gene_symbol": "ASB16-AS1",
  "term_id": "UNKNOWN:0002",
  "gene": "UniProtKB:Q495Z4",
  "term_label": "Unknown biological process"
}